{
  "gene": "UniProtKB:Q8IYI6",
  "term_id": "GO:0000145",
  "gene_name": "Exocyst complex component 8",
  "term_label": "exocyst",
  "gene_symbol": "EXOC8"
}